{
  "term_label": "melanin biosynthetic process",
  "gene_symbol": "OCA2",
  "gene_name": "P protein",
  "gene": "UniProtKB:Q04671",
  "term_id": "GO:0042438"
}